glucarolactone O-hydroxycinnamoyltransferase activity [GO:0047171] (molecular function) Relationships: is_a O-hydroxycinnamoyltransferase activity [GO:0050737] Definition: Catalysis of the reaction: glucarolactone + sinapoyl-CoA = O-sinapoylglucarolactone + CoA. Also known as: sinapoyl-CoA:glucarolactone O-(hydroxycinnamoyl)transferase activity Sources: EC:2.3.1.132, MetaCyc:2.3.1.132-RXN